{
  "gene": "UniProtKB:Q9BZM2",
  "gene_name": "Group IIF secretory phospholipase A2",
  "term_id": "GO:0005543",
  "term_label": "phospholipid binding",
  "gene_symbol": "PLA2G2F"
}